{
  "term_label": "cytoplasm",
  "term_id": "GO:0005737",
  "gene_symbol": "FEZ2",
  "gene": "UniProtKB:Q9UHY8",
  "gene_name": "Fasciculation and elongation protein zeta-2"
}